{
  "gene_symbol": "NDUFAB1",
  "term_id": "GO:0000035",
  "gene_name": "Acyl carrier protein, mitochondrial",
  "gene": "UniProtKB:O14561",
  "term_label": "acyl binding"
}